{
  "term_id": "GO:0140410",
  "gene_name": "Zinc transporter ZIP12",
  "gene_symbol": "SLC39A12",
  "gene": "UniProtKB:Q504Y0",
  "term_label": "monoatomic cation:bicarbonate symporter activity"
}